positive regulation of response to alcohol [GO:1901421] (biological process) Definition: Any process that activates or increases the frequency, rate or extent of response to alcohol. Sources: GOC:TermGenie, GOC:mengo_curators Also known as: up regulation of response to alcohol, up-regulation of response to alcohol, upregulation of response to alcohol, activation of response to alcohol Relationships: is a type of positive regulation of response to stimulus [GO:0048584]; is a type of GO:1901419; positively regulates response to alcohol [GO:0097305] Subtypes: positive regulation of response to ethanol [GO:1901418], GO:1901447, positive regulation of response to butan-1-ol [GO:1901450], positive regulation of cellular response to alcohol [GO:1905959]